postsynaptic intermediate filament cytoskeleton [GO:0099160] (cellular component) References: PMID:25869803 Sources: GOC:dos Definition: The intermediate filament cytoskeleton that is part of a postsynapse. Relationships: is a type of GO:0045111; is a type of postsynaptic cytoskeleton [GO:0099571]